{
  "gene": "UniProtKB:Q9Y6B7",
  "term_id": "UNKNOWN:0001",
  "gene_name": "AP-4 complex subunit beta-1",
  "gene_symbol": "AP4B1",
  "term_label": "Unknown molecular function"
}